{
  "gene_name": "E3 ubiquitin-protein ligase RNF170",
  "term_id": "UNKNOWN:0001",
  "term_label": "Unknown molecular function",
  "gene_symbol": "RNF170",
  "gene": "UniProtKB:Q96K19"
}